{
  "gene_name": "Small integral membrane protein 17",
  "term_label": "Unknown molecular function",
  "gene": "UniProtKB:P0DL12",
  "gene_symbol": "SMIM17",
  "term_id": "UNKNOWN:0001"
}